positive regulation of pulmonary blood vessel remodeling [GO:1905111] (biological process) References: PMID:22161164 Sources: GOC:BHF, GOC:BHF_miRNA, GOC:TermGenie, GOC:bc, GO_REF:0000058 Also known as: positive regulation of pulmonary blood vessel remodelling, up regulation of pulmonary blood vessel remodeling, up-regulation of pulmonary blood vessel remodeling, upregulation of pulmonary blood vessel remodeling, activation of pulmonary blood vessel remodeling Relationships: is a type of regulation of pulmonary blood vessel remodeling [GO:1905109]; is a type of positive regulation of blood vessel remodeling [GO:2000504]; positively regulates GO:0101010 Definition: Any process that activates or increases the frequency, rate or extent of pulmonary blood vessel remodeling.